behavioral fear response [GO:0001662] (biological process) References: PMID:9920659 Sources: GOC:dph Also known as: behavioural fear response Definition: An acute behavioral change resulting from a perceived external threat. Regulation: RO_0002211 by regulation of behavioral fear response [GO:2000822]; negatively regulated by negative regulation of behavioral fear response [GO:2000986]; RO_0002213 by positive regulation of behavioral fear response [GO:2000987] Relationships: is a type of GO:0002209; is a type of fear response [GO:0042596]